regulation of binding [GO:0051098] (BP) Subtypes: regulation of protein binding [GO:0043393], positive regulation of binding [GO:0051099], GO:0051100, regulation of DNA binding [GO:0051101], GO:1901876, GO:1902415 Definition: Any process that modulates the frequency, rate or extent of binding, the selective interaction of a molecule with one or more specific sites on another molecule. Sources: GOC:ai Relationships: is a type of regulation of molecular function [GO:0065009]; regulates GO:0005488